{
  "gene_symbol": "BAG3",
  "term_id": "GO:0005634",
  "gene_name": "BAG family molecular chaperone regulator 3",
  "gene": "UniProtKB:O95817",
  "term_label": "nucleus"
}